methionine-importing ABC transporter complex [GO:1990197] (cellular component) Definition: An ATP-binding cassette (ABC) transporter complex that is capable of methionine-importing activity. An example is the bacterial MetNIQ methionine transporter, that consists of the dimeric ATPase subunit MetN located at the cytoplasmic side of the plasma membrane and the dimeric transmembrane subunit MetI. MetQ is regarded as the periplasmic methionine-binding chaperon subunit, and is capable of transporting methionine from the periplasm into the cytoplasm in an ATP-dependent manner. Relationships: is a type of ATP-binding cassette (ABC) transporter complex [GO:0043190]; is a type of methionine-importing complex [GO:1902509] Also known as: methionine transport complex, methionine transporter complex, methionine transporter complex, ATP-dependent, ATP-binding cassette (ABC) methionine importer complex, ATP-dependent methionine importer complex, ATP-dependent methionine importing complex, ATP-dependent methionine-importing complex, MetNI complex, MetNI transport complex, MetNI transporter complex, MetNIQ complex, MetNIQ transport complex, MetNI transporter, MetNIQ transporter, MetNIQ transporter complex, methionine transporter References: PMID:22095702 Sources: GOC:bhm